siderophore biosynthetic process [GO:0019290] (biological process) References: PMID:20376388 Relationships: is a type of GO:0009237; is a type of GO:0019184; is a type of secondary metabolite biosynthetic process [GO:0044550] Also known as: siderophore anabolism, siderophore biosynthesis, siderophore formation, siderophore synthesis, siderochrome biosynthesis, siderochrome biosynthetic process, siderophore biosynthetic process, peptide formation, siderophore biosynthetic process, peptide modification Regulation: regulated by regulation of siderophore biosynthetic process [GO:1900704]; negatively regulated by GO:1900705; positively regulated by positive regulation of siderophore biosynthetic process [GO:1900706] Subtypes: pyoverdine biosynthetic process [GO:0002049], hydroxymate-containing siderophore biosynthetic process [GO:0019539], catechol-containing siderophore biosynthetic process [GO:0019540], chrysobactin biosynthetic process [GO:0042858], achromobactin biosynthetic process [GO:0042861], pyochelin biosynthetic process [GO:0042864], GO:0140614 Definition: The chemical reactions and pathways resulting in the formation of siderophores, low molecular weight Fe(III)-chelating substances made by aerobic or facultatively anaerobic bacteria, especially when growing under iron deficient conditions. The complexes of Fe(3+)-siderophores have very high stability constants and are taken up by specific transport systems by microorganisms; the subsequent release of iron requires enzymatic action.